{
  "term_label": "pheromone binding",
  "gene": "UniProtKB:Q8TDU5",
  "gene_name": "Putative vomeronasal receptor-like protein 4",
  "gene_symbol": "VN1R17P",
  "term_id": "GO:0005550"
}